{
  "gene_name": "Mitochondrial carrier protein SCaMC-3L",
  "term_id": "GO:0015867",
  "gene_symbol": "SLC25A41",
  "gene": "UniProtKB:Q8N5S1",
  "term_label": "ATP transport"
}